{
  "term_label": "DNA-binding transcription factor activity",
  "gene_symbol": "PKNOX1",
  "term_id": "GO:0003700",
  "gene_name": "Homeobox protein PKNOX1",
  "gene": "UniProtKB:P55347"
}